{
  "term_label": "Unknown biological process",
  "gene_name": "SH3 domain-binding protein 2",
  "gene": "UniProtKB:P78314",
  "term_id": "UNKNOWN:0002",
  "gene_symbol": "SH3BP2"
}